{
  "term_id": "UNKNOWN:0003",
  "gene": "UniProtKB:Q8NI32",
  "gene_name": "Ly6_PLAUR domain-containing protein 6B",
  "term_label": "Unknown cellular component",
  "gene_symbol": "LYPD6B"
}